{
  "gene_symbol": "CETN3",
  "term_id": "GO:0005509",
  "term_label": "calcium ion binding",
  "gene": "UniProtKB:O15182",
  "gene_name": "Centrin-3"
}